{
  "term_id": "UNKNOWN:0003",
  "gene_symbol": "HEXA-AS1",
  "gene": "UniProtKB:Q9H8Q6",
  "gene_name": "Putative uncharacterized protein encoded by HEXA-AS1",
  "term_label": "Unknown cellular component"
}